lymphocyte proliferation [GO:0046651] (biological process) Definition: The expansion of a lymphocyte population by cell division. Sources: GOC:ai Relationships: is a type of GO:0032943; is a type of lymphocyte activation [GO:0046649] Subtypes: natural killer cell proliferation [GO:0001787], T cell proliferation [GO:0042098], GO:0042100 Regulation: regulated by regulation of lymphocyte proliferation [GO:0050670]; positively regulated by GO:0050671; negatively regulated by GO:0050672